{
  "gene_symbol": "S100A7L2",
  "term_label": "calcium-dependent protein binding",
  "gene": "UniProtKB:Q5SY68",
  "gene_name": "Protein S100-A7-like 2",
  "term_id": "GO:0048306"
}